phosphatidylinositol 3-kinase catalytic subunit binding [GO:0036313] (molecular function) Definition: Binding to the catalytic subunit of a phosphatidylinositol 3-kinase. The catalytic subunit catalyzes the addition of a phosphate group to an inositol lipid at the 3' position of the inositol ring. References: PMID:17475214 Sources: GOC:bf Relationships: is a type of kinase binding [GO:0019900]; is a type of GO:0043548 Also known as: PI3K catalytic subunit binding, p110 binding